ferritin complex [GO:0070288] (cellular component) Definition: A protein complex that binds iron and acts as a major iron storage system. There are three major subclasses of ferritins: the classical ferritins (Ftn), the heme-containing bacterioferritins (Bfr) and the DNA-binding proteins from starved cells (Dps). Ftn and Bfr are made of 24 subunits, whereas Dps are smaller with 12 subunits. Ftn is found in most kindoms, while Bfr and Dps are restricted to prokaryotes. Relationships: is a type of protein-containing complex [GO:0032991] References: PMID:19154717, PMID:33881539